{
  "gene_symbol": "EMILIN3",
  "term_id": "UNKNOWN:0003",
  "term_label": "Unknown cellular component",
  "gene": "UniProtKB:Q9NT22",
  "gene_name": "EMILIN-3"
}